negative regulation of fatty acid metabolic process [GO:0045922] (BP) Subtypes: negative regulation of fatty acid biosynthetic process [GO:0045717], negative regulation of fatty acid oxidation [GO:0046322], negative regulation of palmitic acid catabolic process [GO:0106394], negative regulation of methane biosynthetic process from 3-(methylthio)propionic acid [GO:1900334], negative regulation of butyryl-CoA catabolic process to butanol [GO:1900498] Definition: Any process that stops, prevents, or reduces the frequency, rate or extent of the chemical reactions and pathways involving fatty acids. Relationships: is a type of regulation of fatty acid metabolic process [GO:0019217]; is a type of GO:0045833; is a type of GO:0062014; RO_0002212 fatty acid metabolic process [GO:0006631] Sources: GOC:go_curators Also known as: down regulation of fatty acid metabolic process, down-regulation of fatty acid metabolic process, downregulation of fatty acid metabolic process, negative regulation of fatty acid metabolism, inhibition of fatty acid metabolic process